{
  "term_label": "glutathione dehydrogenase (ascorbate) activity",
  "gene_symbol": "GSTO2",
  "gene_name": "Glutathione S-transferase omega-2",
  "gene": "UniProtKB:Q9H4Y5",
  "term_id": "GO:0045174"
}